{
  "gene_name": "Testis-specific Y-encoded-like protein 2",
  "term_id": "UNKNOWN:0002",
  "gene": "UniProtKB:Q9H2G4",
  "gene_symbol": "TSPYL2",
  "term_label": "Unknown biological process"
}